regulation of endocardial cushion to mesenchymal transition involved in heart valve formation [GO:2000800] (biological process) Definition: Any process that modulates the frequency, rate or extent of endocardial cushion to mesenchymal transition involved in heart valve formation. Sources: GOC:BHF Also known as: regulation of endocardial cushion to mesenchymal transition involved in valve formation Relationships: is a type of regulation of endocardial cushion to mesenchymal transition [GO:0140049]; regulates endocardial cushion to mesenchymal transition involved in heart valve formation [GO:0003199] Subtypes: GO:2000801, GO:2000802